positive regulation of cell volume [GO:0045795] (biological process) Relationships: is a type of GO:0006884 Sources: GOC:go_curators Definition: Any process that increases cell volume.